{
  "gene_symbol": "EMC3",
  "term_id": "GO:0071816",
  "gene_name": "ER membrane protein complex subunit 3",
  "term_label": "tail-anchored membrane protein insertion into ER membrane",
  "gene": "UniProtKB:Q9P0I2"
}